diacylglycerol O-acyltransferase activity [GO:0004144] (molecular function) Also known as: 1,2-diacylglycerol acyltransferase activity, acyl-CoA:1,2-diacylglycerol O-acyltransferase activity, diacylglycerol acyltransferase activity, diglyceride O-acyltransferase activity, diglyceride acyltransferase activity, palmitoyl-CoA-sn-1,2-diacylglycerol acyltransferase activity Sources: EC:2.3.1.20 Definition: Catalysis of the reaction: acyl-CoA + 1,2-diacylglycerol = CoA + triacylglycerol. Relationships: is a type of acylglycerol O-acyltransferase activity [GO:0016411]